{
  "gene_name": "T cell receptor beta variable 18",
  "gene_symbol": "TRBV18",
  "term_label": "cell surface receptor signaling pathway",
  "gene": "UniProtKB:A0A087X0M5",
  "term_id": "GO:0007166"
}